{
  "term_id": "GO:0034727",
  "term_label": "piecemeal microautophagy of the nucleus",
  "gene_symbol": "ATG12",
  "gene_name": "Ubiquitin-like protein ATG12",
  "gene": "UniProtKB:O94817"
}